{
  "term_label": "protein-arginine deiminase activity",
  "gene_symbol": "PADI1",
  "gene_name": "Protein-arginine deiminase type-1",
  "gene": "UniProtKB:Q9ULC6",
  "term_id": "GO:0004668"
}